DnaA-L2 complex [GO:1990082] (cellular component) Definition: A protein complex that inhibits unwinding of DNA at the origin of replication and assembly of the pre-primosome. In E. coli, this complex is composed of DnaA and of the ribosomal protein L2. Relationships: is a type of replication inhibiting complex [GO:1990078] References: PMID:21288885 Sources: GOC:bhm